{
  "gene_symbol": "XCL2",
  "gene_name": "Cytokine SCM-1 beta",
  "term_id": "GO:0006954",
  "term_label": "inflammatory response",
  "gene": "UniProtKB:Q9UBD3"
}